{
  "gene": "UniProtKB:P50876",
  "gene_name": "E3 ubiquitin-protein ligase RNF144A",
  "gene_symbol": "RNF144A",
  "term_id": "GO:0005737",
  "term_label": "cytoplasm"
}